{
  "gene": "UniProtKB:Q9NSY2",
  "term_id": "UNKNOWN:0003",
  "gene_name": "StAR-related lipid transfer protein 5",
  "term_label": "Unknown cellular component",
  "gene_symbol": "STARD5"
}